{
  "gene_name": "Dihydrofolate reductase",
  "term_label": "dihydrofolate metabolic process",
  "gene_symbol": "DHFR",
  "gene": "UniProtKB:P00374",
  "term_id": "GO:0046452"
}